{
  "gene": "UniProtKB:Q9NX14",
  "gene_name": "NADH dehydrogenase [ubiquinone] 1 beta subcomplex subunit 11, mitochondrial",
  "term_id": "GO:0045271",
  "gene_symbol": "NDUFB11",
  "term_label": "respiratory chain complex I"
}